{
  "term_label": "protein serine/threonine phosphatase inhibitor activity",
  "gene_name": "PPP2R1A-PPP2R2A-interacting phosphatase regulator 1",
  "gene_symbol": "PABIR1",
  "gene": "UniProtKB:Q96E09",
  "term_id": "GO:0004865"
}